{
  "term_label": "Unknown molecular function",
  "gene_name": "Tenomodulin",
  "gene_symbol": "TNMD",
  "term_id": "UNKNOWN:0001",
  "gene": "UniProtKB:Q9H2S6"
}